ecdysteroid 2-hydroxylase activity [GO:0042768] (molecular function) References: PMID:12177427 Relationships: is_a steroid hydroxylase activity [GO:0008395]; is a type of oxidoreductase activity, acting on paired donors, with incorporation or reduction of molecular oxygen, reduced iron-sulfur protein as one donor, and incorporation of one atom of oxygen [GO:0016713] Definition: Catalysis of the hydroxylation of an ecdysteroid at carbon position 2. Note: Note that in the ecdysteroidogenic pathway, this activity catalyzes the conversion of 2-deoxyecdysone to ecdysone. It can also catalyze the conversion of 2,22-dideoxyecdysone (ketotriol) to 22-deoxyecdysone.